{
  "term_label": "nucleus",
  "gene_symbol": "SREBF1",
  "gene": "UniProtKB:P36956",
  "term_id": "GO:0005634",
  "gene_name": "Sterol regulatory element-binding protein 1"
}